cellular response to water deprivation [GO:0042631] (biological process) Definition: Any process that results in a change in state or activity of a cell (in terms of movement, secretion, enzyme production, gene expression, etc.) as a result of deprivation of water. Sources: GOC:go_curators Also known as: cellular response to drought Relationships: is a type of response to water deprivation [GO:0009414]; is a type of GO:0033554; is a type of cellular response to water stimulus [GO:0071462] Subtypes: GO:0071465